skeletal muscle tissue regeneration [GO:0043403] (BP) Relationships: is a type of tissue regeneration [GO:0042246] Regulation: positively regulated by positive regulation of skeletal muscle tissue regeneration [GO:0043415]; regulated by regulation of skeletal muscle tissue regeneration [GO:0043416]; negatively regulated by negative regulation of skeletal muscle tissue regeneration [GO:0043417] Subtypes: skeletal muscle regeneration at neuromuscular junction [GO:0014730] References: PMID:12021255, PMID:16607119 Sources: GOC:ef, GOC:mtg_muscle Also known as: myofiber turnover Definition: The regrowth of skeletal muscle tissue to repair injured or damaged muscle fibers in the postnatal stage.